{
  "gene_symbol": "TENM3",
  "gene_name": "Teneurin-3",
  "term_id": "GO:0048666",
  "gene": "UniProtKB:Q9P273",
  "term_label": "neuron development"
}